2-carene synthase activity [GO:0102702] (molecular function) References: PMID:10700382 Sources: GOC:pz Relationships: is a type of carbon-oxygen lyase activity, acting on phosphates [GO:0016838] Definition: Catalysis of the reaction: geranyl diphosphate = (+)-2-carene + diphosphoric acid.